phosphatidylserine transfer activity [GO:0140343] (molecular function) Also known as: intermembrane phosphatidylserine carrier activity Relationships: is_a phospholipid transfer activity [GO:0120014] Definition: Removes phosphatidylserine from the outer leaflet of a donor membrane, transports it through the aqueous phase while protected in a hydrophobic pocket, and brings it to the outer leaflet of an acceptor membrane. References: PMID:26206935 Subtypes: phosphatidylserine-phosphatidylinositol-4-phosphate exchange activity [GO:0160270]